{
  "gene_name": "Probable G-protein coupled receptor 156",
  "term_id": "GO:0004965",
  "gene_symbol": "GPR156",
  "gene": "UniProtKB:Q8NFN8",
  "term_label": "G protein-coupled GABA receptor activity"
}